{
  "term_label": "sno(s)RNA catabolic process",
  "gene": "UniProtKB:Q96DE0",
  "term_id": "GO:0016077",
  "gene_symbol": "NUDT16",
  "gene_name": "U8 snoRNA-decapping enzyme"
}